response to chloramphenicol [GO:1901322] (biological process) Definition: Any process that results in a change in state or activity of a cell or an organism (in terms of movement, secretion, enzyme production, gene expression, etc.) as a result of a chloramphenicol stimulus. Subtypes: GO:0072747 Relationships: is a type of GO:1901698; is a type of GO:1901700 Sources: GOC:TermGenie